{
  "term_label": "regulation of blood vessel endothelial cell migration",
  "gene_name": "Lysosomal Pro-X carboxypeptidase",
  "gene": "UniProtKB:P42785",
  "term_id": "GO:0043535",
  "gene_symbol": "PRCP"
}